{
  "gene_name": "Keratin, type II cytoskeletal 6C",
  "term_id": "GO:0031424",
  "term_label": "keratinization",
  "gene": "UniProtKB:P48668",
  "gene_symbol": "KRT6C"
}